{
  "gene_symbol": "ZNF516",
  "term_id": "GO:0000978",
  "gene": "UniProtKB:Q92618",
  "gene_name": "Zinc finger protein 516",
  "term_label": "RNA polymerase II cis-regulatory region sequence-specific DNA binding"
}